{
  "gene_name": "Phospholipid phosphatase 4",
  "term_label": "phospholipid dephosphorylation",
  "gene": "UniProtKB:Q5VZY2",
  "gene_symbol": "PLPP4",
  "term_id": "GO:0046839"
}